{
  "gene_name": "Uncharacterized protein C2orf15",
  "term_id": "UNKNOWN:0003",
  "gene_symbol": "C2orf15",
  "term_label": "Unknown cellular component",
  "gene": "UniProtKB:Q8WU43"
}